open form four-way junction DNA binding [GO:0000401] (molecular function) Definition: Binding to a DNA segment containing the open form of a four-way junction, also known as a Holliday junction, a structure where two DNA double strands are held together by reciprocal exchange of two of the four strands, one strand each from the two original helices. The open form of a four-way junction can be diagrammed without any of the strands crossing over. Also known as: open form Holliday junction binding References: PMID:15563464 Sources: GOC:krc, ISBN:0815332181 Relationships: is a type of four-way junction DNA binding [GO:0000400]